{
  "term_id": "UNKNOWN:0002",
  "gene_symbol": "JPT1",
  "gene_name": "Jupiter microtubule associated homolog 1",
  "gene": "UniProtKB:Q9UK76",
  "term_label": "Unknown biological process"
}